{
  "gene_symbol": "TRBJ2-2P",
  "gene": "UniProtKB:A0A0A0MTA2",
  "gene_name": "T cell receptor beta joining 2-2P (non-functional) (Fragment)",
  "term_label": "Unknown biological process",
  "term_id": "UNKNOWN:0002"
}